{
  "gene_name": "Putative HLA class I histocompatibility antigen, alpha chain H",
  "term_id": "GO:0002486",
  "gene_symbol": "HLA-H",
  "gene": "UniProtKB:P01893",
  "term_label": "antigen processing and presentation of endogenous peptide antigen via MHC class I via ER pathway, TAP-independent"
}